{
  "term_label": "cytoplasm",
  "gene": "UniProtKB:A6NES4",
  "term_id": "GO:0005737",
  "gene_symbol": "MROH2A",
  "gene_name": "Maestro heat-like repeat-containing protein family member 2A"
}